azobenzene reductase (NADP+) activity [GO:0050446] (molecular function) Definition: Catalysis of the reaction: aniline + N,N-dimethyl-1,4-phenylenediamine + 2 NADP+ = 4-(dimethylamino)azobenzene + 2 H+ + 2 NADPH. Also known as: NADPH-dependent azoreductase activity, azo reductase activity, azo-dye reductase activity, azoreductase activity, NC-reductase activity, New coccine (NC)-reductase activity, methyl red azoreductase activity, orange I azoreductase activity, orange II azoreductase activity, N,N-dimethyl-1,4-phenylenediamine, aniline:NADP+ oxidoreductase activity, N,N-dimethyl-4-phenylazoaniline azoreductase activity, NAD(P)H:1-(4'-sulfophenylazo)-2-naphthol oxidoreductase activity, NADPH2-dependent azoreductase activity, NADPH2:4-(dimethylamino)azobenzene oxidoreductase activity, NADPH:4-(dimethylamino)azobenzene oxidoreductase activity, dibromopropylaminophenylazobenzoic azoreductase activity, dimethylaminobenzene reductase activity, new coccine (NC)-reductase, nicotinamide adenine dinucleotide (phosphate) azoreductase activity, p-aminoazobenzene reductase activity, p-dimethylaminoazobenzene azoreductase activity Relationships: is_a GO:0046857 Sources: RHEA:16269